methylnaphthalene catabolic process [GO:0043635] (biological process) Relationships: is a type of GO:0042178 References: PMID:16535687 Sources: GOC:jl Definition: The chemical reactions and pathways resulting in the breakdown of methylnaphthalene, an organic compound, C10H7CH3, obtained from coal tar. Also known as: 1-methylnaphthalene catabolic process, 1-methylnaphthalene catabolism, 2-methylnaphthalene catabolic process, 2-methylnaphthalene catabolism, 1-MN catabolic process, 1-MN catabolism, 2-MN catabolic process, 2-MN catabolism